{
  "gene_symbol": "METTL13",
  "term_label": "protein-lysine N-methyltransferase activity",
  "term_id": "GO:0016279",
  "gene_name": "eEF1A lysine and N-terminal methyltransferase",
  "gene": "UniProtKB:Q8N6R0"
}